{
  "gene_symbol": "BAZ1A",
  "term_id": "GO:0003677",
  "term_label": "DNA binding",
  "gene": "UniProtKB:Q9NRL2",
  "gene_name": "Bromodomain adjacent to zinc finger domain protein 1A"
}